sulfite reductase (ferredoxin) activity [GO:0050311] (molecular function) Sources: EC:1.8.7.1, MetaCyc:SULFITE-REDUCTASE-FERREDOXIN-RXN Relationships: is a type of oxidoreductase activity, acting on a sulfur group of donors, iron-sulfur protein as acceptor [GO:0016673] Also known as: sulphite reductase (ferredoxin) activity, ferredoxin-sulfite reductase activity, hydrogen-sulfide:ferredoxin oxidoreductase activity Definition: Catalysis of the reaction: hydrogen sulfide + 3 oxidized ferredoxin + 3 H2O = sulfite + 3 reduced ferredoxin.